{
  "gene_name": "N-myc proto-oncogene protein",
  "gene": "UniProtKB:P04198",
  "term_label": "DNA-binding transcription factor activity, RNA polymerase II-specific",
  "gene_symbol": "MYCN",
  "term_id": "GO:0000981"
}